{
  "gene_symbol": "PPP5C",
  "term_label": "nucleus",
  "gene": "UniProtKB:P53041",
  "gene_name": "Serine_threonine-protein phosphatase 5",
  "term_id": "GO:0005634"
}